skeletal muscle tissue growth [GO:0048630] (BP) Relationships: is a type of GO:0048589; is part of skeletal muscle tissue development [GO:0007519] References: PMID:15726494, PMID:15907921 Sources: GOC:lm Definition: The increase in size or mass of a skeletal muscle. This may be due to a change in the fiber number or size. Regulation: regulated by regulation of skeletal muscle tissue growth [GO:0048631]; negatively regulated by negative regulation of skeletal muscle tissue growth [GO:0048632]; RO_0002213 by positive regulation of skeletal muscle tissue growth [GO:0048633]